{
  "gene": "UniProtKB:O75387",
  "term_label": "Unknown cellular component",
  "term_id": "UNKNOWN:0003",
  "gene_name": "Large neutral amino acids transporter small subunit 3",
  "gene_symbol": "SLC43A1"
}